{
  "term_label": "regulation of transcription by RNA polymerase II",
  "term_id": "GO:0006357",
  "gene_symbol": "IRX5",
  "gene_name": "Iroquois-class homeodomain protein IRX-5",
  "gene": "UniProtKB:P78411"
}